{
  "term_id": "GO:0045095",
  "gene_name": "Keratin, type I cytoskeletal 23",
  "term_label": "keratin filament",
  "gene": "UniProtKB:Q9C075",
  "gene_symbol": "KRT23"
}